{
  "gene_name": "Zinc finger protein 132",
  "gene_symbol": "ZNF132",
  "term_label": "RNA polymerase II cis-regulatory region sequence-specific DNA binding",
  "gene": "UniProtKB:P52740",
  "term_id": "GO:0000978"
}